{
  "gene": "UniProtKB:P05062",
  "term_id": "GO:0030388",
  "gene_symbol": "ALDOB",
  "gene_name": "Fructose-bisphosphate aldolase B",
  "term_label": "fructose 1,6-bisphosphate metabolic process"
}